{
  "term_id": "UNKNOWN:0003",
  "gene_name": "Putative uncharacterized protein MGC34800",
  "term_label": "Unknown cellular component",
  "gene": "UniProtKB:Q8N6K4",
  "gene_symbol": "Q8N6K4"
}